{
  "term_label": "nucleolus",
  "term_id": "GO:0005730",
  "gene_name": "Probable ATP-dependent RNA helicase DDX27",
  "gene": "UniProtKB:Q96GQ7",
  "gene_symbol": "DDX27"
}